{
  "gene": "UniProtKB:Q93083",
  "gene_symbol": "MT1L",
  "term_id": "GO:0071276",
  "gene_name": "Metallothionein-1L",
  "term_label": "cellular response to cadmium ion"
}